{
  "gene_name": "Coiled-coil domain-containing protein 80",
  "gene_symbol": "CCDC80",
  "term_id": "UNKNOWN:0001",
  "term_label": "Unknown molecular function",
  "gene": "UniProtKB:Q76M96"
}